{
  "term_label": "Unknown biological process",
  "gene_name": "Transmembrane protein 202",
  "term_id": "UNKNOWN:0002",
  "gene_symbol": "TMEM202",
  "gene": "UniProtKB:A6NGA9"
}